{
  "gene_name": "Transmembrane protein 165",
  "term_id": "GO:0005794",
  "gene_symbol": "TMEM165",
  "term_label": "Golgi apparatus",
  "gene": "UniProtKB:Q9HC07"
}